{
  "gene": "UniProtKB:Q9Y5E1",
  "gene_name": "Protocadherin beta-9",
  "term_id": "GO:0050839",
  "gene_symbol": "PCDHB9",
  "term_label": "cell adhesion molecule binding"
}